{
  "gene_symbol": "SLCO1B3-SLCO1B7",
  "gene": "UniProtKB:F5H094",
  "gene_name": "SLCO1B3-SLCO1B7 readthrough transcript protein",
  "term_id": "GO:0015125",
  "term_label": "bile acid transmembrane transporter activity"
}